{
  "gene_name": "Guanine nucleotide-binding protein G(i) subunit alpha-2",
  "gene_symbol": "GNAI2",
  "term_id": "GO:0001664",
  "term_label": "G protein-coupled receptor binding",
  "gene": "UniProtKB:P04899"
}